{
  "term_label": "alpha-mannosidase activity",
  "gene_symbol": "MAN2B2",
  "term_id": "GO:0004559",
  "gene_name": "Epididymis-specific alpha-mannosidase",
  "gene": "UniProtKB:Q9Y2E5"
}